{
  "term_label": "nervous system development",
  "term_id": "GO:0007399",
  "gene": "UniProtKB:Q8IZ57",
  "gene_name": "Neurensin-1",
  "gene_symbol": "NRSN1"
}